positive regulation of glial cell-derived neurotrophic factor receptor signaling pathway involved in ureteric bud formation [GO:2000735] (biological process) Sources: GOC:obol Also known as: positive regulation of GDNF receptor signaling pathway of ureteric bud formation, positive regulation of glial cell derived neurotrophic factor receptor signaling pathway of ureteric bud formation, positive regulation of glial cell line-derived neurotrophic factor receptor signalling pathway of ureteric bud formation, positive regulation of glial cell-derived neurotrophic factor receptor signaling pathway of ureteric bud formation, positive regulation of glial cell-derived neurotrophic factor receptor signalling pathway of ureteric bud formation Definition: Any process that activates or increases the frequency, rate or extent of glial cell-derived neurotrophic factor receptor signaling pathway involved in ureteric bud formation. Relationships: is a type of positive regulation of signal transduction [GO:0009967]; is a type of GO:2000733; RO_0002213 glial cell-derived neurotrophic factor receptor signaling pathway involved in ureteric bud formation [GO:2000701]